leukocyte activation involved in inflammatory response [GO:0002269] (biological process) Subtypes: microglial cell activation [GO:0001774] Relationships: is a type of leukocyte activation [GO:0045321]; is part of inflammatory response [GO:0006954] Sources: GOC:add, ISBN:0781735149 Definition: A change in the morphology or behavior of a leukocyte resulting from exposure to an activating factor such as a cellular or soluble ligand, leading to the initiation or perpetuation of an inflammatory response. Also known as: immune cell activation during inflammatory response, leukocyte activation during inflammatory response